{
  "term_label": "Unknown biological process",
  "term_id": "UNKNOWN:0002",
  "gene_name": "Serine_arginine repetitive matrix protein 3",
  "gene": "UniProtKB:A6NNA2",
  "gene_symbol": "SRRM3"
}